{
  "gene": "UniProtKB:P14653",
  "term_label": "regulation of transcription by RNA polymerase II",
  "term_id": "GO:0006357",
  "gene_name": "Homeobox protein Hox-B1",
  "gene_symbol": "HOXB1"
}